positive regulation of chitin-based cuticle tanning [GO:0045801] (biological process) Sources: GOC:go_curators, GOC:jid, GOC:mtg_sensu Also known as: positive regulation of cuticle tanning, up regulation of cuticle tanning, up-regulation of cuticle tanning, upregulation of cuticle tanning, activation of cuticle tanning, positive regulation of cuticle hardening, stimulation of cuticle tanning Subtypes: positive regulation of adult chitin-containing cuticle pigmentation [GO:0048084] Relationships: is a type of regulation of chitin-based cuticle tanning [GO:0007564]; is a type of positive regulation of developmental process [GO:0051094]; is_a GO:0051240; positively regulates chitin-based cuticle sclerotization [GO:0007593] Definition: Any process that activates or increases the frequency, rate or extent of chitin-based cuticular tanning.